{
  "gene_symbol": "CALM2",
  "term_id": "GO:0005513",
  "term_label": "detection of calcium ion",
  "gene": "UniProtKB:P0DP24",
  "gene_name": "Calmodulin-2"
}